hexitol catabolic process [GO:0019407] (biological process) Subtypes: sorbitol catabolic process [GO:0006062], galactitol catabolic process [GO:0019404], mannitol catabolic process [GO:0019592] Also known as: hexitol breakdown, hexitol catabolism, hexitol degradation Relationships: is a type of hexitol metabolic process [GO:0006059]; is a type of alditol catabolic process [GO:0019405] Definition: The chemical reactions and pathways resulting in the breakdown of hexitols, any alditol with a chain of six carbon atoms in the molecule. Sources: ISBN:0198506732